{
  "gene": "UniProtKB:Q96MT0",
  "term_id": "UNKNOWN:0001",
  "gene_name": "Putative uncharacterized protein FLJ31958",
  "term_label": "Unknown molecular function",
  "gene_symbol": "Q96MT0"
}